germarium-derived female germ-line cyst encapsulation [GO:0030708] (biological process) Definition: Formation of a single follicular epithelium around the germ-line derived cells of a cyst formed in the germarium. An example of this process is found in Drosophila melanogaster. References: PMID:11591336 Sources: GOC:mtg_sensu Relationships: is a type of female germ-line cyst encapsulation [GO:0048139]; is part of germarium-derived egg chamber formation [GO:0007293]; is part of follicle cell of egg chamber development [GO:0030707]